{
  "gene_name": "Beta-defensin 114",
  "gene": "UniProtKB:Q30KQ6",
  "term_id": "GO:0042056",
  "term_label": "chemoattractant activity",
  "gene_symbol": "DEFB114"
}